positive regulation of fibrinolysis [GO:0051919] (biological process) Sources: GOC:ai Definition: Any process that activates, maintains or increases the frequency, rate or extent of fibrinolysis, an ongoing process that solubilizes fibrin, resulting in the removal of small blood clots. Also known as: up regulation of fibrinolysis, up-regulation of fibrinolysis, upregulation of fibrinolysis, activation of fibrinolysis, stimulation of fibrinolysis Relationships: is a type of negative regulation of blood coagulation [GO:0030195]; is a type of positive regulation of biological process [GO:0048518]; is a type of GO:0051917; positively regulates GO:0042730